{
  "term_id": "GO:0034987",
  "gene": "UniProtKB:P01854",
  "gene_name": "Immunoglobulin heavy constant epsilon",
  "term_label": "immunoglobulin receptor binding",
  "gene_symbol": "IGHE"
}